{
  "term_label": "Unknown molecular function",
  "gene_symbol": "C9orf153",
  "gene_name": "Uncharacterized protein C9orf153",
  "term_id": "UNKNOWN:0001",
  "gene": "UniProtKB:Q5TBE3"
}